{
  "term_label": "mRNA binding",
  "term_id": "GO:0003729",
  "gene": "UniProtKB:P0DJD4",
  "gene_symbol": "RBMY1C",
  "gene_name": "RNA-binding motif protein, Y chromosome, family 1 member C"
}